histone H3K4 deacetylase activity, hydrolytic mechanism [GO:1990162] (molecular function) Also known as: histone H3K14 deacetylase activity, histone deacetylase activity (H3-K4 specific), histone H3-K4 deacetylase activity Definition: Catalysis of the reaction: histone H3 N6-acetyl-L-lysine (position 4) + H2O = histone H3 L-lysine (position 4) + acetate. This reaction represents the removal of an acetyl group from lysine at position 4 of the histone H3 protein. Relationships: is_a histone H3K deacetylase activity [GO:0141050]; is a type of GO:0141221 References: PMID:23771057, PMID:28450737 Sources: GOC:al Note: Comment: Note that the residue position corresponds to the canonical human H3 histone (UniProtKB:P84243); this residue is conserved across all eukaryotes. Residue 1 is the first residue following removal of the initiating Methionine (Met). Note that each histone is encoded by multiple genes, and sequences may vary across different genes within an organism.